{
  "term_id": "GO:0045835",
  "gene_symbol": "FBXO5",
  "gene": "UniProtKB:Q9UKT4",
  "term_label": "negative regulation of meiotic nuclear division",
  "gene_name": "F-box only protein 5"
}